{
  "gene_symbol": "ZNF572",
  "term_id": "GO:0000978",
  "gene_name": "Zinc finger protein 572",
  "gene": "UniProtKB:Q7Z3I7",
  "term_label": "RNA polymerase II cis-regulatory region sequence-specific DNA binding"
}